{
  "gene": "UniProtKB:Q96P66",
  "term_label": "positive regulation of MAPK cascade",
  "gene_symbol": "GPR101",
  "term_id": "GO:0043410",
  "gene_name": "Probable G-protein coupled receptor 101"
}